{
  "term_label": "Unknown molecular function",
  "term_id": "UNKNOWN:0001",
  "gene": "UniProtKB:Q9BRK4",
  "gene_name": "Leucine zipper putative tumor suppressor 2",
  "gene_symbol": "LZTS2"
}